{
  "term_id": "GO:0007186",
  "gene_name": "Guanine nucleotide-binding protein G(I)_G(S)_G(O) subunit gamma-5B",
  "term_label": "G protein-coupled receptor signaling pathway",
  "gene": "UniProtKB:A0A804HLA8",
  "gene_symbol": "GNG5B"
}